{
  "term_label": "prostaglandin metabolic process",
  "gene_name": "Aldo-keto reductase family 1 member C4",
  "gene": "UniProtKB:P17516",
  "gene_symbol": "AKR1C4",
  "term_id": "GO:0006693"
}